{
  "gene_symbol": "CDK7",
  "gene": "UniProtKB:P50613",
  "gene_name": "Cyclin-dependent kinase 7",
  "term_label": "cyclin-dependent protein serine/threonine kinase activity",
  "term_id": "GO:0004693"
}